ribosome assembly [GO:0042255] (biological process) Subtypes: cytosolic ribosome assembly [GO:0042256], GO:0061668 Relationships: is a type of membraneless organelle assembly [GO:0140694]; is part of ribosome biogenesis [GO:0042254] Definition: The aggregation, arrangement and bonding together of the mature ribosome and of its subunits. Also known as: ribosomal subunit assembly References: PMID:30467428 Sources: GOC:ma